positive regulation of pole plasm oskar mRNA localization [GO:0045856] (biological process) Definition: Any process that activates or increases the frequency, rate or extent of the process in which oskar mRNA is transported to, or maintained in, the oocyte pole plasm. Also known as: positive regulation of oocyte pole plasm oskar mRNA localization, positive regulation of pole plasm oskar mRNA localisation, up regulation of pole plasm oskar mRNA localization, up-regulation of pole plasm oskar mRNA localization, upregulation of pole plasm oskar mRNA localization, activation of pole plasm oskar mRNA localization, stimulation of pole plasm oskar mRNA localization Relationships: is a type of regulation of pole plasm oskar mRNA localization [GO:0007317]; is a type of GO:1904582; positively regulates pole plasm oskar mRNA localization [GO:0045451] Sources: GOC:go_curators